{
  "gene": "UniProtKB:Q9H8X9",
  "term_label": "protein targeting to membrane",
  "term_id": "GO:0006612",
  "gene_name": "Palmitoyltransferase ZDHHC11",
  "gene_symbol": "ZDHHC11"
}